{
  "gene_symbol": "YIPF7",
  "gene": "UniProtKB:Q8N8F6",
  "term_label": "endoplasmic reticulum to Golgi vesicle-mediated transport",
  "term_id": "GO:0006888",
  "gene_name": "Protein YIPF7"
}